{
  "term_id": "UNKNOWN:0003",
  "gene_name": "Suppressor of cytokine signaling 7",
  "gene": "UniProtKB:O14512",
  "gene_symbol": "SOCS7",
  "term_label": "Unknown cellular component"
}